{
  "gene": "UniProtKB:P43652",
  "term_id": "GO:0031667",
  "term_label": "response to nutrient levels",
  "gene_symbol": "AFM",
  "gene_name": "Afamin"
}